{
  "term_label": "endoplasmic reticulum tubular network organization",
  "gene": "UniProtKB:Q9BRK0",
  "gene_symbol": "REEP2",
  "term_id": "GO:0071786",
  "gene_name": "Receptor expression-enhancing protein 2"
}